{
  "gene_name": "EKC_KEOPS complex subunit TPRKB",
  "gene": "UniProtKB:Q9Y3C4",
  "term_label": "EKC/KEOPS complex",
  "gene_symbol": "TPRKB",
  "term_id": "GO:0000408"
}